{
  "gene_symbol": "FOXO4",
  "gene": "UniProtKB:P98177",
  "term_id": "GO:0005634",
  "gene_name": "Forkhead box protein O4",
  "term_label": "nucleus"
}